{
  "term_label": "mitochondrion",
  "gene": "UniProtKB:Q9NTK1",
  "gene_name": "Protein DEPP1",
  "gene_symbol": "DEPP1",
  "term_id": "GO:0005739"
}